{
  "term_id": "GO:0019901",
  "gene": "UniProtKB:Q9C035",
  "gene_name": "Tripartite motif-containing protein 5",
  "gene_symbol": "TRIM5",
  "term_label": "protein kinase binding"
}